ABC-type thiosulfate transporter activity [GO:0102025] (molecular function) Sources: GOC:mlg, GOC:pz Also known as: thiosulphate ABC transporter activity, ATPase-coupled thiosulfate transmembrane transporter activity, thiosulfate transmembrane-transporting ATPase activity Relationships: is a type of GO:0015117; is a type of ABC-type transporter activity [GO:0140359] Definition: Enables the transfer of a solute or solutes from one side of a membrane to the other according to the reaction: ATP + H2O + thiosulfate(out) = ADP + phosphate + thiosulfate(in).